{
  "term_id": "UNKNOWN:0003",
  "gene_symbol": "TAGLN",
  "term_label": "Unknown cellular component",
  "gene_name": "Transgelin",
  "gene": "UniProtKB:Q01995"
}